{
  "term_id": "UNKNOWN:0001",
  "term_label": "Unknown molecular function",
  "gene_symbol": "WDR46",
  "gene": "UniProtKB:O15213",
  "gene_name": "WD repeat-containing protein 46"
}